{
  "gene_name": "Cadherin-related family member 2",
  "gene": "UniProtKB:Q9BYE9",
  "term_id": "GO:0030855",
  "gene_symbol": "CDHR2",
  "term_label": "epithelial cell differentiation"
}